{
  "term_label": "Unknown cellular component",
  "gene_name": "Protein FAM240C",
  "gene": "UniProtKB:A0A1B0GVR7",
  "gene_symbol": "FAM240C",
  "term_id": "UNKNOWN:0003"
}